negative regulation of D-aspartate import across plasma membrane [GO:0140216] (biological process) References: PMID:27663541 Definition: Any process that stops, prevents or reduces the frequency, rate or extent of the directed import of D-aspartate from the extracellular region across the plasma membrane and into the cytosol. Relationships: is a type of negative regulation of organic acid transport [GO:0032891]; is a type of negative regulation of transmembrane transport [GO:0034763]; is a type of negative regulation of amino acid transport [GO:0051956]; is a type of regulation of D-aspartate import across plasma membrane [GO:0140215]; negatively regulates D-aspartate import across plasma membrane [GO:0070779]